{
  "gene_symbol": "PLEC",
  "gene": "UniProtKB:Q15149",
  "term_id": "GO:0030056",
  "term_label": "hemidesmosome",
  "gene_name": "Plectin"
}